collecting duct development [GO:0072044] (biological process) Sources: GOC:mtg_kidney_jan10 Subtypes: GO:0061211, outer medullary collecting duct development [GO:0072060], inner medullary collecting duct development [GO:0072061], metanephric collecting duct development [GO:0072205] Definition: The process whose specific outcome is the progression of a collecting duct over time, from its formation to the mature structure. The collecting duct responds to vasopressin and aldosterone to regulate water, electrolyte and acid-base balance. It is the final common path through which urine flows before entering the ureter and then emptying into the bladder. Relationships: is a type of GO:0035295; is part of GO:0001822